hypoxanthine dehydrogenase activity [GO:0070674] (molecular function) Also known as: hypoxanthine oxidoreductase activity, NAD-hypoxanthine dehydrogenase activity, hypoxanthine-NAD oxidoreductase activity, hypoxanthine/NAD(+) oxidoreductase activity, hypoxanthine/NAD+ oxidoreductase activity, hypoxanthine:NAD+ oxidoreductase activity Sources: GOC:mah, GOC:pde Definition: Catalysis of the reaction: hypoxanthine + NAD+ + H2O = xanthine + NADH + H+. Relationships: is_a oxidoreductase activity, acting on CH or CH2 groups, NAD or NADP as acceptor [GO:0016726]